{
  "term_id": "UNKNOWN:0002",
  "term_label": "Unknown biological process",
  "gene": "UniProtKB:P55082",
  "gene_symbol": "MFAP3",
  "gene_name": "Microfibril-associated glycoprotein 3"
}